{
  "term_label": "metalloaminopeptidase activity",
  "gene_symbol": "METAP1",
  "gene": "UniProtKB:P53582",
  "term_id": "GO:0070006",
  "gene_name": "Methionine aminopeptidase 1"
}